response to metal ion starvation [GO:0180055] (biological process) References: PMID:24024382 Relationships: is a type of response to starvation [GO:0042594] Definition: Any process that results in a change in state or activity of a cell or an organism (in terms of movement, secretion, enzyme production, gene expression, etc.) as a result of a starvation stimulus, deprivation of some metal ion. Subtypes: response to manganese ion starvation [GO:0090551], response to copper ion starvation [GO:0120126], response to zinc ion starvation [GO:0120127], response to iron ion starvation [GO:1990641]